{
  "gene_symbol": "DYSF",
  "gene": "UniProtKB:O75923",
  "gene_name": "Dysferlin",
  "term_id": "GO:0005509",
  "term_label": "calcium ion binding"
}